{
  "gene_name": "Protein Wnt-8b",
  "gene": "UniProtKB:Q93098",
  "gene_symbol": "WNT8B",
  "term_label": "cell fate commitment",
  "term_id": "GO:0045165"
}